{
  "gene_name": "Autophagy-related protein 2 homolog A",
  "term_label": "pexophagy",
  "term_id": "GO:0000425",
  "gene": "UniProtKB:Q2TAZ0",
  "gene_symbol": "ATG2A"
}